{
  "term_id": "GO:0005200",
  "gene": "UniProtKB:P61158",
  "term_label": "structural constituent of cytoskeleton",
  "gene_symbol": "ACTR3",
  "gene_name": "Actin-related protein 3"
}